deactivation of mitotic spindle assembly checkpoint [GO:1902426] (biological process) References: PMID:19075002, PMID:19592249 Sources: GOC:TermGenie, GOC:dph, GOC:vw Also known as: down regulation of mitotic cell cycle spindle assembly checkpoint, down regulation of mitotic spindle assembly checkpoint, down-regulation of mitotic cell cycle spindle assembly checkpoint, down-regulation of mitotic spindle assembly checkpoint, downregulation of mitotic cell cycle spindle assembly checkpoint, downregulation of mitotic spindle assembly checkpoint, negative regulation of mitotic cell cycle spindle assembly checkpoint, negative regulation of mitotic spindle assembly checkpoint, mitotic spindle assembly checkpoint silencing, mitotic spindle assembly deactivation, down regulation of Mad2-dependent checkpoint, down-regulation of Mad2-dependent checkpoint, downregulation of Mad2-dependent checkpoint, inhibition of Mad2-dependent checkpoint, inhibition of mitotic cell cycle spindle assembly checkpoint, inhibition of mitotic spindle assembly checkpoint, negative regulation of Mad2-dependent checkpoint Note: A mitotic spindle assembly checkpoint is either activated or switched off; no other means of reducing the frequency, rate or extent of this process are currently known. Definition: A positive regulation of the mitotic metaphase/anaphase transition that results from deactivation of the mitotic spindle assembly checkpoint. Relationships: is a type of negative regulation of mitotic spindle assembly checkpoint signaling [GO:0140499]